{
  "gene_name": "Microtubule-associated protein 9",
  "gene": "UniProtKB:Q49MG5",
  "term_id": "GO:1902412",
  "term_label": "regulation of mitotic cytokinesis",
  "gene_symbol": "MAP9"
}